dGMP binding [GO:0032565] (MF) Relationships: is a type of guanyl deoxyribonucleotide binding [GO:0032560]; is a type of anion binding [GO:0043168] Sources: GOC:mah Definition: Binding to dGMP, deoxyguanosine monophosphate.